{
  "term_id": "GO:0045040",
  "gene_symbol": "MTX3",
  "gene": "UniProtKB:Q5HYI7",
  "gene_name": "Metaxin-3",
  "term_label": "protein insertion into mitochondrial outer membrane"
}